{
  "gene_name": "Platelet-derived growth factor receptor beta",
  "term_id": "GO:0007169",
  "term_label": "cell surface receptor protein tyrosine kinase signaling pathway",
  "gene_symbol": "PDGFRB",
  "gene": "UniProtKB:P09619"
}